{
  "gene_symbol": "TRAF1",
  "gene": "UniProtKB:Q13077",
  "term_id": "GO:0005737",
  "term_label": "cytoplasm",
  "gene_name": "TNF receptor-associated factor 1"
}